{
  "gene": "UniProtKB:O75828",
  "gene_name": "Carbonyl reductase [NADPH] 3",
  "term_label": "carbonyl reductase (NADPH) activity",
  "term_id": "GO:0004090",
  "gene_symbol": "CBR3"
}